{
  "gene_name": "Zinc-regulated GTPase metalloprotein activator 1F",
  "gene": "UniProtKB:Q4V339",
  "gene_symbol": "ZNG1F",
  "term_id": "GO:0051604",
  "term_label": "protein maturation"
}